{
  "term_id": "GO:0006417",
  "gene": "UniProtKB:Q15397",
  "term_label": "regulation of translation",
  "gene_name": "Pumilio homolog 3",
  "gene_symbol": "PUM3"
}